{
  "term_id": "UNKNOWN:0003",
  "gene": "UniProtKB:A0A0B4J245",
  "term_label": "Unknown cellular component",
  "gene_name": "T cell receptor alpha variable 12-1",
  "gene_symbol": "TRAV12-1"
}